protein C inhibitor-plasma kallikrein complex [GO:0036030] (cellular component) References: PMID:2844223, PMID:8536714 Sources: GOC:ans Definition: A heterodimeric protein complex that contains protein C inhibitor (SERPINA5) and plasma kallikrein (KLK1B); formation of the complex inhibits the serine protease activity of plasma kallikrein. Also known as: PCI-plasma kallikrein complex, SERPINA5-plasma kallikrein complex, plasma serine protease inhibitor-plasma kallikrein complex, protein C inhibitor-KLKB1 complex, serpin A5-plasma kallikrein complex Relationships: is a type of serine protease inhibitor complex [GO:0097180]